type 2 fibroblast growth factor receptor binding [GO:0005111] (molecular function) Also known as: FGFR2 binding, heartless binding, FGFR2 ligand, heartless ligand, type 2 fibroblast growth factor receptor ligand Note: Note that heartless is the Drosophila gene encoding the type 2 fibroblast growth factor receptor (FGFR2). Definition: Binding to a type 2 fibroblast growth factor receptor (FGFR2). Relationships: is a type of fibroblast growth factor receptor binding [GO:0005104] Sources: GOC:fb_curators